{
  "term_label": "riboflavin kinase activity",
  "gene": "UniProtKB:Q969G6",
  "gene_symbol": "RFK",
  "gene_name": "Riboflavin kinase",
  "term_id": "GO:0008531"
}